{
  "gene": "UniProtKB:Q5TC82",
  "gene_symbol": "RC3H1",
  "term_id": "GO:0035613",
  "term_label": "RNA stem-loop binding",
  "gene_name": "Roquin-1"
}